{
  "term_label": "Unknown cellular component",
  "gene_symbol": "MPPED1",
  "gene": "UniProtKB:O15442",
  "gene_name": "Metallophosphoesterase domain-containing protein 1",
  "term_id": "UNKNOWN:0003"
}